{
  "gene_name": "YEATS domain-containing protein 2",
  "gene": "UniProtKB:Q9ULM3",
  "term_label": "nucleus",
  "gene_symbol": "YEATS2",
  "term_id": "GO:0005634"
}